{
  "term_label": "endomembrane system",
  "gene_symbol": "RAB19",
  "gene_name": "Ras-related protein Rab-19",
  "gene": "UniProtKB:A4D1S5",
  "term_id": "GO:0012505"
}